{
  "gene": "UniProtKB:Q9H1Z9",
  "term_label": "Unknown biological process",
  "term_id": "UNKNOWN:0002",
  "gene_name": "Tetraspanin-10",
  "gene_symbol": "TSPAN10"
}